{
  "term_id": "UNKNOWN:0001",
  "gene": "UniProtKB:A6NKF1",
  "term_label": "Unknown molecular function",
  "gene_name": "SAC3 domain-containing protein 1",
  "gene_symbol": "SAC3D1"
}